{
  "gene_symbol": "C3orf70",
  "term_id": "UNKNOWN:0001",
  "gene_name": "UPF0524 protein C3orf70",
  "term_label": "Unknown molecular function",
  "gene": "UniProtKB:A6NLC5"
}